negative regulation of cell cycle phase transition [GO:1901988] (biological process) Subtypes: cell cycle checkpoint signaling [GO:0000075], negative regulation of mitotic cell cycle phase transition [GO:1901991], negative regulation of meiotic cell cycle phase transition [GO:1901994], negative regulation of metaphase/anaphase transition of cell cycle [GO:1902100], negative regulation of cell cycle G2/M phase transition [GO:1902750], GO:1902807 Also known as: down regulation of cell cycle phase transition, down regulation of cell cycle transition, down-regulation of cell cycle phase transition, down-regulation of cell cycle transition, downregulation of cell cycle phase transition, downregulation of cell cycle transition, inhibition of cell cycle transition, negative regulation of cell cycle transition, inhibition of cell cycle phase transition References: PMID:22841721 Sources: GOC:TermGenie, GOC:mtg_cell_cycle Definition: Any process that stops, prevents or reduces the frequency, rate or extent of cell cycle phase transition. Relationships: is a type of negative regulation of cell cycle process [GO:0010948]; is a type of GO:1901987; negatively regulates cell cycle phase transition [GO:0044770]